{
  "term_id": "GO:0004222",
  "gene_name": "Collagenase 3",
  "term_label": "metalloendopeptidase activity",
  "gene": "UniProtKB:P45452",
  "gene_symbol": "MMP13"
}